{
  "gene_name": "Phospholipase A and acyltransferase 1",
  "term_id": "GO:0016410",
  "gene": "UniProtKB:Q9HDD0",
  "gene_symbol": "PLAAT1",
  "term_label": "N-acyltransferase activity"
}